{
  "term_id": "GO:0016020",
  "gene_symbol": "TOM1L1",
  "gene": "UniProtKB:O75674",
  "gene_name": "TOM1-like protein 1",
  "term_label": "membrane"
}